glutathione dehydrogenase (ascorbate) activity [GO:0045174] (molecular function) Definition: Catalysis of the reaction: dehydroascorbate + 2 glutathione = L-ascorbate + glutathione disulfide. Sources: RHEA:24424 Also known as: dehydroascorbate reductase activity, DHA reductase activity, GDOR, dehydroascorbic acid reductase activity, dehydroascorbic reductase activity, glutathione dehydroascorbate reductase activity, glutathione:dehydroascorbate oxidoreductase activity, glutathione:dehydroascorbic acid oxidoreductase activity Relationships: is a type of glutathione disulfide oxidoreductase activity [GO:0015038]; is_a antioxidant activity [GO:0016209]; is a type of oxidoreductase activity, acting on a sulfur group of donors, quinone or similar compound as acceptor [GO:0016672]